transepithelial chloride transport [GO:0030321] (biological process) Definition: The directed movement of chloride ions from one side of an epithelium to the other. Relationships: is a type of chloride transport [GO:0006821]; is a type of GO:0070633 Sources: GOC:mah